{
  "gene_symbol": "GGT2P",
  "term_id": "GO:0031179",
  "gene_name": "Inactive glutathione hydrolase 2",
  "gene": "UniProtKB:P36268",
  "term_label": "peptide modification"
}